{
  "term_id": "UNKNOWN:0002",
  "gene_symbol": "CABP7",
  "gene_name": "Calcium-binding protein 7",
  "gene": "UniProtKB:Q86V35",
  "term_label": "Unknown biological process"
}